negative regulation of meiotic DNA double-strand break formation [GO:1903342] (biological process) Also known as: down regulation of meiotic DNA double-strand break formation, down-regulation of meiotic DNA double-strand break formation, downregulation of meiotic DNA double-strand break formation, inhibition of meiotic DNA double-strand break formation Subtypes: GO:1905262 Definition: Any process that stops, prevents or reduces the frequency, rate or extent of meiotic DNA double-strand break formation. Relationships: is a type of negative regulation of cell cycle process [GO:0010948]; is_a GO:0051053; is a type of regulation of meiotic DNA double-strand break formation [GO:1903341]; is a type of negative regulation of reproductive process [GO:2000242]; negatively regulates meiotic DNA double-strand break formation [GO:0042138] References: PMID:25103240 Sources: GOC:TermGenie, GO_REF:0000058